ligand-gated monoatomic ion channel activity [GO:0015276] (molecular function) Definition: Enables the transmembrane transfer of an ion by a channel that opens when a specific ligand has been bound by the channel complex or one of its constituent parts. Sources: GOC:mtg_transport, ISBN:0815340729 Also known as: ligand-gated ion channel activity, ionotropic receptor activity Relationships: is a type of monoatomic ion channel activity [GO:0005216]; is_a ligand-gated channel activity [GO:0022834] Subtypes: intracellularly ligand-gated monoatomic ion channel activity [GO:0005217], GO:0005230, cyclic nucleotide-activated monoatomic ion channel activity [GO:0043855], GO:0099094, ligand-gated monoatomic anion channel activity [GO:0099095], ligand-gated monoatomic ion channel activity involved in regulation of presynaptic membrane potential [GO:0099507], pH-gated monoatomic ion channel activity [GO:0160128], ionotropic olfactory receptor activity [GO:0170020], ionotropic taste receptor activity [GO:0170021]